{
  "term_label": "DNA repair",
  "gene_name": "E3 ubiquitin-protein ligase FANCL",
  "gene": "UniProtKB:Q9NW38",
  "gene_symbol": "FANCL",
  "term_id": "GO:0006281"
}